lung field specification [GO:0060424] (biological process) Regulation: positively regulated by GO:0060492 Relationships: is a type of GO:0010092; is a type of foregut regionalization [GO:0060423]; is part of primary lung bud formation [GO:0060431] Also known as: lung specification Definition: The process that results in the delineation of a specific region of the foregut into the area in which the lung will develop. Sources: GOC:dph, GOC:mtg_lung